{
  "term_label": "olfactory receptor activity",
  "gene": "UniProtKB:Q8NG75",
  "gene_symbol": "OR5T1",
  "term_id": "GO:0004984",
  "gene_name": "Olfactory receptor 5T1"
}